{
  "gene_name": "Heterochromatin protein 1-binding protein 3",
  "term_id": "GO:0005694",
  "gene_symbol": "HP1BP3",
  "gene": "UniProtKB:Q5SSJ5",
  "term_label": "chromosome"
}